{
  "gene_symbol": "RELA",
  "term_id": "GO:0038061",
  "gene": "UniProtKB:Q04206",
  "gene_name": "Transcription factor p65",
  "term_label": "non-canonical NF-kappaB signal transduction"
}